2-hydroxy-1,4-benzoxazin-3-one monooxygenase activity [GO:0036193] (molecular function) Definition: Catalysis of the reaction: 2-hydroxy-2H-1,4-benzoxazin-3(4H)-one + O2 + reduced [NADPH--hemoprotein reductase] = DIBOA + H+ + H2O + oxidized [NADPH--hemoprotein reductase]. Relationships: is_a oxidoreductase activity, acting on paired donors, with incorporation or reduction of molecular oxygen, reduced flavin or flavoprotein as one donor, and incorporation of one atom of oxygen [GO:0016712] Sources: RHEA:31939